{
  "gene_symbol": "SOX9",
  "term_id": "GO:0000981",
  "gene_name": "Transcription factor SOX-9",
  "term_label": "DNA-binding transcription factor activity, RNA polymerase II-specific",
  "gene": "UniProtKB:P48436"
}